{
  "gene_name": "Adenosine 3'-phospho 5'-phosphosulfate transporter 2",
  "term_label": "3'-phosphoadenosine 5'-phosphosulfate transmembrane transporter activity",
  "gene_symbol": "SLC35B3",
  "term_id": "GO:0046964",
  "gene": "UniProtKB:Q9H1N7"
}